positive regulation of cell cycle checkpoint [GO:1901978] (biological process) References: PMID:23028116 Sources: GOC:TermGenie, GOC:mtg_cell_cycle Relationships: is_a regulation of cell cycle checkpoint [GO:1901976]; is a type of GO:1902533; positively regulates cell cycle checkpoint signaling [GO:0000075] Subtypes: GO:0090232, GO:2000003 Also known as: up regulation of cell cycle checkpoint, up-regulation of cell cycle checkpoint, upregulation of cell cycle checkpoint, activation of cell cycle checkpoint, positive regulation of G1/S checkpoint, positive regulation of G1/S transition checkpoint Definition: Any process that activates or increases the frequency, rate or extent of cell cycle checkpoint.